{
  "gene_symbol": "TRGV11",
  "term_label": "Unknown cellular component",
  "gene": "UniProtKB:A0A075B6L2",
  "gene_name": "Probable non-functional T cell receptor gamma variable 11",
  "term_id": "UNKNOWN:0003"
}